{
  "gene": "UniProtKB:Q8TBB6",
  "gene_name": "Probable cationic amino acid transporter",
  "gene_symbol": "SLC7A14",
  "term_id": "GO:0006865",
  "term_label": "amino acid transport"
}